{
  "gene": "UniProtKB:P51828",
  "term_id": "GO:0005886",
  "term_label": "plasma membrane",
  "gene_name": "Adenylate cyclase type 7",
  "gene_symbol": "ADCY7"
}